{
  "gene_symbol": "HK3",
  "term_id": "GO:0006006",
  "term_label": "glucose metabolic process",
  "gene": "UniProtKB:P52790",
  "gene_name": "Hexokinase-3"
}